{
  "gene_name": "BMP-2-inducible protein kinase",
  "term_id": "GO:0019208",
  "gene": "UniProtKB:Q9NSY1",
  "term_label": "phosphatase regulator activity",
  "gene_symbol": "BMP2K"
}